sensory perception of hot stimulus [GO:0062036] (biological process) Definition: The series of events required for an organism to receive a hot temperature stimulus, convert it to a molecular signal, and recognize and characterize the signal. Relationships: is a type of thermoception [GO:0050955] References: PMID:21335241